{
  "term_id": "GO:0051402",
  "term_label": "neuron apoptotic process",
  "gene_name": "Diablo IAP-binding mitochondrial protein",
  "gene_symbol": "DIABLO",
  "gene": "UniProtKB:Q9NR28"
}